{
  "term_label": "ventricular cardiac muscle cell action potential",
  "term_id": "GO:0086005",
  "gene_name": "Potassium voltage-gated channel subfamily E member 1",
  "gene": "UniProtKB:P15382",
  "gene_symbol": "KCNE1"
}